negative regulation of granulocyte chemotaxis [GO:0071623] (biological process) Relationships: is a type of negative regulation of leukocyte chemotaxis [GO:0002689]; is a type of GO:0071622; negatively regulates granulocyte chemotaxis [GO:0071621] Sources: GOC:mah Subtypes: negative regulation of neutrophil chemotaxis [GO:0090024], negative regulation of eosinophil chemotaxis [GO:2000423] Definition: Any process that decreases the rate, frequency or extent of granulocyte chemotaxis. Granulocyte chemotaxis is the movement of a granulocyte in response to an external stimulus.